{
  "term_id": "GO:0005634",
  "term_label": "nucleus",
  "gene": "UniProtKB:Q9Y5J3",
  "gene_symbol": "HEY1",
  "gene_name": "Hairy_enhancer-of-split related with YRPW motif protein 1"
}